alternative mRNA splicing, via spliceosome [GO:0000380] (biological process) Definition: The process of generating multiple mRNA molecules from a given set of exons by differential use of exons from the primary transcript(s) to form multiple mature mRNAs that vary in their exon composition. Subtypes: mRNA alternative trans-splicing [GO:0000366] Note: Note that this process most commonly occurs in cis, selecting or skipping exons from the same primary transcript, but it has also been observed to occur in trans at low frequency, at least in some mammals. References: PMID:12110900 Sources: GOC:krc Relationships: is a type of mRNA splicing, via spliceosome [GO:0000398] Also known as: splice site selection, alternative nuclear mRNA splicing, via spliceosome Regulation: regulated by regulation of alternative mRNA splicing, via spliceosome [GO:0000381]